{
  "gene_symbol": "TESK2",
  "term_label": "protein serine/threonine kinase activity",
  "gene_name": "Dual specificity testis-specific protein kinase 2",
  "gene": "UniProtKB:Q96S53",
  "term_id": "GO:0004674"
}